{
  "gene": "UniProtKB:Q8N960",
  "term_label": "centrosome",
  "gene_symbol": "CEP120",
  "term_id": "GO:0005813",
  "gene_name": "Centrosomal protein of 120 kDa"
}